{
  "term_label": "neuronal signal transduction",
  "term_id": "GO:0023041",
  "gene_symbol": "MACO1",
  "gene_name": "Macoilin",
  "gene": "UniProtKB:Q8N5G2"
}